{
  "term_id": "GO:0005777",
  "gene_symbol": "EPHX2",
  "term_label": "peroxisome",
  "gene_name": "Bifunctional epoxide hydrolase 2",
  "gene": "UniProtKB:P34913"
}